{
  "gene_symbol": "PPIH",
  "term_id": "GO:0006457",
  "gene_name": "Peptidyl-prolyl cis-trans isomerase H",
  "term_label": "protein folding",
  "gene": "UniProtKB:O43447"
}